{
  "gene_name": "Transmembrane protein 272",
  "term_label": "Unknown biological process",
  "gene": "UniProtKB:A0A1B0GTI8",
  "term_id": "UNKNOWN:0002",
  "gene_symbol": "TMEM272"
}